positive regulation of leukocyte mediated immunity [GO:0002705] (BP) Sources: GOC:add Definition: Any process that activates or increases the frequency, rate, or extent of leukocyte mediated immunity. Relationships: is a type of positive regulation of immune effector process [GO:0002699]; is a type of GO:0002703; positively regulates GO:0002443 Subtypes: GO:0001912, positive regulation of lymphocyte mediated immunity [GO:0002708], GO:0002732, GO:0002888 Also known as: positive regulation of immune cell mediated immunity, positive regulation of leucocyte mediated immunity, up regulation of leukocyte mediated immunity, up-regulation of leukocyte mediated immunity, upregulation of leukocyte mediated immunity, activation of leukocyte mediated immunity, stimulation of leukocyte mediated immunity